regulation of protein targeting [GO:1903533] (biological process) Also known as: regulation of protein sorting along secretory pathway, regulation of nascent polypeptide association Subtypes: regulation of protein targeting to membrane [GO:0090313], regulation of protein targeting to mitochondrion [GO:1903214], regulation of protein targeting to vacuole involved in autophagy [GO:1904051], GO:2001159 Sources: GOC:TermGenie, GO_REF:0000058 Definition: Any process that modulates the frequency, rate or extent of protein targeting. Relationships: is a type of regulation of establishment of protein localization [GO:0070201]; regulates GO:0006605